{
  "gene": "UniProtKB:Q8NGE8",
  "term_id": "GO:0004984",
  "term_label": "olfactory receptor activity",
  "gene_name": "Olfactory receptor 4D9",
  "gene_symbol": "OR4D9"
}